{
  "gene": "UniProtKB:P22001",
  "gene_name": "Potassium voltage-gated channel subfamily A member 3",
  "term_label": "action potential",
  "term_id": "GO:0001508",
  "gene_symbol": "KCNA3"
}